{
  "gene_name": "Transmembrane protein 183A",
  "term_id": "UNKNOWN:0002",
  "gene_symbol": "TMEM183A",
  "gene": "UniProtKB:Q8IXX5",
  "term_label": "Unknown biological process"
}